hexagonal collagen network of basement membrane [GO:0140155] (cellular component) References: PMID:21421911, PMID:2376131, PMID:3047147, PMID:31387942 Relationships: is a type of collagen network [GO:0098645]; is part of GO:0140143 Definition: Supramolecular structure formed by trimers of collagen VIII and found in the basement membrane.